{
  "gene_name": "ATP synthase subunit ATP5MJ, mitochondrial",
  "gene": "UniProtKB:P56378",
  "term_id": "UNKNOWN:0001",
  "term_label": "Unknown molecular function",
  "gene_symbol": "ATP5MJ"
}